retinal cone cell fate specification [GO:0042672] (biological process) Definition: The process in which a cell becomes capable of differentiating autonomously into a retinal cone cell in an environment that is neutral with respect to the developmental pathway; upon specification, the cell fate can be reversed. Regulation: negatively regulated by negative regulation of retinal cone cell fate specification [GO:0009998]; regulated by GO:0042673 Sources: GOC:go_curators Relationships: is a type of GO:0043704; is part of retinal cone cell fate commitment [GO:0046551]